{
  "gene_name": "Probable C-mannosyltransferase DPY19L3",
  "gene": "UniProtKB:Q6ZPD9",
  "term_id": "GO:0005789",
  "gene_symbol": "DPY19L3",
  "term_label": "endoplasmic reticulum membrane"
}